induction of synaptic vesicle exocytosis by positive regulation of presynaptic cytosolic calcium ion concentration [GO:0099703] (biological process) Relationships: is a type of GO:0099171; is a type of positive regulation of presynaptic cytosolic calcium concentration [GO:0099533]; is a type of GO:2000302; is part of chemical synaptic transmission [GO:0007268] Definition: The induction of synaptic vesicle release by any process that leads to a rise in intracellular calcium ion concentration at the presynapse. This is the first step in synaptic transmission. Sources: GOC:dos, ISBN:9780071120005